{
  "gene_name": "Uncharacterized protein C8orf58",
  "gene": "UniProtKB:Q8NAV2",
  "term_label": "Unknown biological process",
  "term_id": "UNKNOWN:0002",
  "gene_symbol": "C8orf58"
}